{
  "gene": "UniProtKB:Q9HAW0",
  "gene_name": "Transcription factor IIIB 50 kDa subunit",
  "term_id": "GO:0097550",
  "gene_symbol": "BRF2",
  "term_label": "transcription preinitiation complex"
}